{
  "term_id": "GO:0071947",
  "gene_symbol": "OTUD7A",
  "gene_name": "OTU domain-containing protein 7A",
  "term_label": "protein deubiquitination involved in ubiquitin-dependent protein catabolic process",
  "gene": "UniProtKB:Q8TE49"
}